{
  "term_label": "protein N-terminal-serine acetyltransferase activity",
  "gene_name": "N-alpha-acetyltransferase 10",
  "gene": "UniProtKB:P41227",
  "term_id": "GO:1990189",
  "gene_symbol": "NAA10"
}